negative regulation of cytoplasmic translational initiation [GO:1904689] (biological process) Subtypes: negative regulation of formation of translation preinitiation complex [GO:1901194], negative regulation of cap-dependent translational initiation [GO:1903675], GO:1903678, negative regulation of cytoplasmic translational initiation in response to stress [GO:1990625] References: PMID:12242291 Sources: GOC:TermGenie, GO_REF:0000058 Definition: Any process that stops, prevents or reduces the frequency, rate or extent of cytoplasmic translational initiation. Relationships: is a type of GO:0045947; is a type of regulation of cytoplasmic translational initiation [GO:1904688]; negatively regulates cytoplasmic translational initiation [GO:0002183] Also known as: down regulation of cytoplasmic translational initiation, down-regulation of cytoplasmic translational initiation, downregulation of cytoplasmic translational initiation, inhibition of cytoplasmic translational initiation